{
  "gene_name": "Casein kinase II subunit beta",
  "gene": "UniProtKB:P67870",
  "gene_symbol": "CSNK2B",
  "term_id": "GO:0005956",
  "term_label": "protein kinase CK2 complex"
}